{
  "term_label": "gamma-aminobutyric acid signaling pathway",
  "gene": "UniProtKB:P14867",
  "gene_name": "Gamma-aminobutyric acid receptor subunit alpha-1",
  "gene_symbol": "GABRA1",
  "term_id": "GO:0007214"
}